{
  "gene_symbol": "FCGR1BP",
  "term_label": "IgG receptor activity",
  "term_id": "GO:0019770",
  "gene": "UniProtKB:Q92637",
  "gene_name": "Putative high affinity immunoglobulin gamma Fc receptor IB"
}